{
  "gene_symbol": "ANKRD20A8P",
  "term_label": "Unknown biological process",
  "term_id": "UNKNOWN:0002",
  "gene_name": "Ankyrin repeat domain-containing protein 20B",
  "gene": "UniProtKB:Q5CZ79"
}